cAMP biosynthetic process [GO:0006171] (biological process) Relationships: is a type of purine ribonucleotide biosynthetic process [GO:0009152]; is a type of GO:0009190; is a type of cAMP metabolic process [GO:0046058] Also known as: 3',5' cAMP biosynthesis, 3',5' cAMP biosynthetic process, 3',5'-cAMP biosynthesis, 3',5'-cAMP biosynthetic process, adenosine 3',5'-cyclophosphate biosynthesis, adenosine 3',5'-cyclophosphate biosynthetic process, cAMP anabolism, cAMP biosynthesis, cAMP formation, cAMP synthesis, cyclic AMP biosynthesis, cyclic AMP biosynthetic process Sources: ISBN:0198506732 Definition: The chemical reactions and pathways resulting in the formation of the nucleotide cAMP (cyclic AMP, adenosine 3',5'-cyclophosphate).